{
  "gene": "UniProtKB:Q5T870",
  "term_id": "UNKNOWN:0003",
  "gene_symbol": "PRR9",
  "term_label": "Unknown cellular component",
  "gene_name": "Proline-rich protein 9"
}